prostaglandin secretion involved in immune response [GO:0090323] (biological process) Relationships: is a type of GO:0032310; is part of immune response [GO:0006955] Note: Note that this term is in the subset of terms that should not be used for direct gene product annotation. Instead, select one of the 'regulation' children terms. Regulation: positively regulated by positive regulation of prostaglandin secretion involved in immune response [GO:0061078] Sources: GOC:dph, GOC:tb Definition: The regulated release of a prostaglandin that contributes to the immune response. Prostaglandins are a group of biologically active metabolites which contain a cyclopentane ring.